{
  "gene_symbol": "EMILIN2",
  "gene_name": "EMILIN-2",
  "gene": "UniProtKB:Q9BXX0",
  "term_label": "Unknown cellular component",
  "term_id": "UNKNOWN:0003"
}